{
  "term_label": "Unknown cellular component",
  "gene_symbol": "FAM25C",
  "gene_name": "Protein FAM25C",
  "term_id": "UNKNOWN:0003",
  "gene": "UniProtKB:B3EWG5"
}